regulation of response to cell cycle checkpoint signaling [GO:1902145] (biological process) Also known as: regulation of cell cycle checkpoint effector process, regulation of response to signal involved in cell cycle checkpoint, regulation of G1/S transition checkpoint effector process, regulation of G2/M transition checkpoint effector process, regulation of response to G1/S transition checkpoint signaling, regulation of response to G2/M transition checkpoint signaling, regulation of response to signal involved in G1/S transition checkpoint, regulation of response to signal involved in G2/M transition checkpoint Relationships: is_a regulation of response to biotic stimulus [GO:0002831]; is a type of GO:0050794; regulates response to cell cycle checkpoint signaling [GO:0072396] Subtypes: positive regulation of response to cell cycle checkpoint signaling [GO:1902146], GO:1902147, GO:1902151 Definition: Any process that modulates the frequency, rate or extent of response to cell cycle checkpoint signaling. Sources: GOC:TermGenie, GOC:mtg_cell_cycle